{
  "gene": "UniProtKB:Q5VWM4",
  "term_label": "Cul2-RING ubiquitin ligase complex",
  "term_id": "GO:0031462",
  "gene_symbol": "PRAMEF8",
  "gene_name": "PRAME family member 8"
}